{
  "gene_symbol": "OXNAD1",
  "term_label": "Unknown biological process",
  "gene": "UniProtKB:Q96HP4",
  "gene_name": "Oxidoreductase NAD-binding domain-containing protein 1",
  "term_id": "UNKNOWN:0002"
}